{
  "gene_name": "Transient receptor potential cation channel subfamily M member 3",
  "gene": "UniProtKB:Q9HCF6",
  "term_label": "monoatomic cation transmembrane transport",
  "gene_symbol": "TRPM3",
  "term_id": "GO:0098655"
}